{
  "gene_name": "Methylmalonic aciduria type A protein, mitochondrial",
  "gene_symbol": "MMAA",
  "term_id": "GO:0005737",
  "term_label": "cytoplasm",
  "gene": "UniProtKB:Q8IVH4"
}